{
  "term_id": "GO:0044183",
  "gene": "UniProtKB:P11021",
  "gene_name": "Endoplasmic reticulum chaperone BiP",
  "gene_symbol": "HSPA5",
  "term_label": "protein folding chaperone"
}